{
  "term_id": "GO:0042102",
  "gene": "UniProtKB:P42081",
  "term_label": "positive regulation of T cell proliferation",
  "gene_symbol": "CD86",
  "gene_name": "T-lymphocyte activation antigen CD86"
}